{
  "term_id": "GO:0034612",
  "gene": "UniProtKB:O15205",
  "term_label": "response to tumor necrosis factor",
  "gene_name": "Ubiquitin D",
  "gene_symbol": "UBD"
}